{
  "term_label": "transcription coregulator activity",
  "term_id": "GO:0003712",
  "gene": "UniProtKB:A2AJT9",
  "gene_symbol": "BCLAF3",
  "gene_name": "BCLAF1 and THRAP3 family member 3"
}